{
  "term_label": "Unknown biological process",
  "gene_name": "Solute carrier family 25 member 35",
  "gene_symbol": "SLC25A35",
  "gene": "UniProtKB:Q3KQZ1",
  "term_id": "UNKNOWN:0002"
}